{
  "gene_name": "Heat shock protein HSP 90-alpha",
  "gene": "UniProtKB:P07900",
  "gene_symbol": "HSP90AA1",
  "term_label": "nucleus",
  "term_id": "GO:0005634"
}